posterior head segmentation [GO:0035289] (biological process) Relationships: is a type of head segmentation [GO:0035287] Also known as: gnathal segmentation References: PMID:15382136 Definition: Partitioning the posterior region of the insect head anlage into gnathal (mandibular, maxillary and labial) segments. Unlike the anterior head (procephalic) segments, formation of the posterior head (gnathal) segments occurs by a similar mechanism to trunk segmentation, where a cascade of gap genes, pair-rule genes and segment-polarity genes subdivide the embryo into progressively smaller domains. Note: See also the fly_anatomy.ontology term 'gnathal segment ; FBbt:00000011' and its children.